tetrahydromethanopterin biosynthetic process [GO:2001118] (biological process) Subtypes: 5,6,7,8-tetrahydromethanopterin biosynthetic process [GO:1901285], 5,6,7,8-tetrahydrosarcinapterin biosynthetic process [GO:1901855] Relationships: is a type of GO:2001116 Also known as: tetrahydromethanopterin biosynthesis Sources: GOC:mengo_curators Definition: The chemical reactions and pathways resulting in the formation of a tetrahydromethanopterin.